{
  "gene_name": "Putative taste receptor type 2 member 33",
  "term_label": "Unknown biological process",
  "gene_symbol": "TAS2R33",
  "gene": "UniProtKB:P0DSN6",
  "term_id": "UNKNOWN:0002"
}